{
  "term_id": "GO:0007229",
  "gene_name": "Integrin beta-6",
  "gene_symbol": "ITGB6",
  "gene": "UniProtKB:P18564",
  "term_label": "integrin-mediated signaling pathway"
}